JUN kinase kinase kinase kinase activity [GO:0042656] (molecular function) Also known as: JUNKKKK activity Relationships: is a type of MAP kinase kinase kinase kinase activity [GO:0008349]; is part of JNK cascade [GO:0007254] Definition: Catalysis of the phosphorylation and activation of JUN kinase kinase kinases (JNKKKs). Sources: GOC:bf